{
  "term_id": "GO:0021686",
  "term_label": "cerebellar granular layer maturation",
  "gene": "UniProtKB:Q8N111",
  "gene_symbol": "CEND1",
  "gene_name": "Cell cycle exit and neuronal differentiation protein 1"
}